{
  "gene": "UniProtKB:Q8ND83",
  "term_id": "GO:0007020",
  "gene_symbol": "SLAIN1",
  "gene_name": "SLAIN motif-containing protein 1",
  "term_label": "microtubule nucleation"
}